regulation of vascular associated smooth muscle cell dedifferentiation [GO:1905174] (biological process) Also known as: regulation of vascular smooth muscle cell dedifferentiation Relationships: is a type of regulation of developmental process [GO:0050793]; is a type of regulation of cellular process [GO:0050794]; regulates vascular associated smooth muscle cell dedifferentiation [GO:1990936] Subtypes: negative regulation of vascular associated smooth muscle cell dedifferentiation [GO:1905175], GO:1905176 References: PMID:19088079 Sources: GOC:BHF, GOC:BHF_miRNA, GOC:TermGenie, GOC:rph, GO_REF:0000058 Definition: Any process that modulates the frequency, rate or extent of vascular smooth muscle cell dedifferentiation.